{
  "term_label": "Unknown cellular component",
  "gene": "UniProtKB:Q9Y6Z5",
  "term_id": "UNKNOWN:0003",
  "gene_symbol": "AFDN-DT",
  "gene_name": "Putative uncharacterized protein AFDN-DT"
}